{
  "term_label": "prostate gland growth",
  "term_id": "GO:0060736",
  "gene": "UniProtKB:Q6NUJ1",
  "gene_name": "Proactivator polypeptide-like 1",
  "gene_symbol": "PSAPL1"
}